{
  "gene_symbol": "TRGV9",
  "term_id": "UNKNOWN:0001",
  "gene": "UniProtKB:Q99603",
  "term_label": "Unknown molecular function",
  "gene_name": "T cell receptor gamma variable 9"
}